{
  "gene_name": "Neuroserpin",
  "term_id": "GO:0005615",
  "gene": "UniProtKB:Q99574",
  "gene_symbol": "SERPINI1",
  "term_label": "extracellular space"
}